(-)-endo-fenchol synthase activity [GO:0050437] (molecular function) Also known as: (-)-endo-fenchol cyclase activity, geranyl pyrophosphate:(-)-endo-fenchol cyclase activity, geranyl-diphosphate diphosphate-lyase [cyclizing, (-)-endo-fenchol-forming] Definition: Catalysis of the reaction: geranyl diphosphate + H2O = (-)-endo-fenchol + diphosphate. Sources: EC:4.2.3.10, RHEA:20565 Relationships: is a type of carbon-oxygen lyase activity, acting on phosphates [GO:0016838]